{
  "gene": "UniProtKB:P18509",
  "term_id": "GO:0043005",
  "gene_symbol": "ADCYAP1",
  "gene_name": "Pituitary adenylate cyclase-activating polypeptide",
  "term_label": "neuron projection"
}